{
  "gene_symbol": "KCTD4",
  "term_id": "UNKNOWN:0002",
  "gene": "UniProtKB:Q8WVF5",
  "gene_name": "BTB_POZ domain-containing protein KCTD4",
  "term_label": "Unknown biological process"
}